{
  "gene": "UniProtKB:Q9Y664",
  "gene_symbol": "KPTN",
  "term_label": "lamellipodium",
  "term_id": "GO:0030027",
  "gene_name": "KICSTOR complex protein kaptin"
}